{
  "term_label": "Unknown molecular function",
  "gene_symbol": "ZNF295-AS1",
  "gene": "UniProtKB:Q8N0V1",
  "gene_name": "Putative uncharacterized protein ZNF295-AS1",
  "term_id": "UNKNOWN:0001"
}